{
  "gene": "UniProtKB:Q9UM00",
  "term_label": "endoplasmic reticulum calcium ion homeostasis",
  "term_id": "GO:0032469",
  "gene_name": "Calcium load-activated calcium channel",
  "gene_symbol": "TMCO1"
}